positive regulation of entry into reproductive diapause [GO:0061965] (BP) Definition: Any process that activates or increases the rate or extent of the dormancy process that results in entry into reproductive diapause. Reproductive diapause is a form of diapause where the organism itself will remain fully active, including feeding and other routine activities, but the reproductive organs experience a tissue-specific reduction in metabolism, with characteristic triggering and releasing stimuli. References: PMID:27689881 Sources: GOC:ha Relationships: is a type of positive regulation of developmental process [GO:0051094]; is a type of GO:0061963; positively regulates GO:0055116